termination of bipolar cell growth [GO:0051520] (biological process) Definition: Any process that stops the active process of bipolar cell growth, polarized growth from both ends of a cell. Sources: GOC:ai Relationships: is a type of negative regulation of bipolar cell growth [GO:0051517]